acyl-lipid omega-3 desaturase (cytochrome b5) activity [GO:0102859] (molecular function) Sources: RHEA:46404 Also known as: 1-18:1-2-18:2-phosphatidylcholine desaturase activity (SN2-18:3 forming) Definition: Catalysis of the reaction: a (9Z,12Z)-octadecadienoyl-containing glycerolipid + 2 Fe(II)-[cytochrome b5] + 2 H+ + O2 = (9Z,12Z,15Z)-octadecatrienoyl-containing glycerolipid + 2 Fe(III)-[cytochrome b5] + 2 H2O. Relationships: is a type of GO:0016717